{
  "gene_name": "Glutathione S-transferase Mu 4",
  "gene_symbol": "GSTM4",
  "term_label": "glutathione transferase activity",
  "gene": "UniProtKB:Q03013",
  "term_id": "GO:0004364"
}